{
  "term_label": "regulation of mitotic spindle organization",
  "gene_name": "Ankyrin repeat domain-containing protein 53",
  "gene": "UniProtKB:Q8N9V6",
  "gene_symbol": "ANKRD53",
  "term_id": "GO:0060236"
}